regulation of mesenchymal to epithelial transition involved in mesonephros morphogenesis [GO:2000084] (biological process) Definition: Any process that modulates the frequency, rate or extent of mesenchymal to epithelial transition involved in mesonephros morphogenesis. Also known as: regulation of mesonephric mesenchyme to epithelial transition Sources: GOC:mtg_kidney_jan10 Subtypes: negative regulation of mesenchymal to epithelial transition involved in mesonephros morphogenesis [GO:2000085], positive regulation of mesenchymal to epithelial transition involved in mesonephros morphogenesis [GO:2000086] Relationships: is a type of regulation of epithelial cell differentiation involved in kidney development [GO:2000696]; regulates mesenchymal to epithelial transition involved in mesonephros morphogenesis [GO:0061261]